{
  "term_label": "extracellular space",
  "gene_symbol": "VEGFA",
  "term_id": "GO:0005615",
  "gene_name": "Vascular endothelial growth factor A, long form",
  "gene": "UniProtKB:P15692"
}